male meiosis II [GO:0007142] (biological process) Definition: A cell cycle process comprising the steps by which a cell progresses through male meiosis II, the second meiotic division in the male germline. Sources: GOC:dph, GOC:mah Also known as: male meiosis II nuclear division Relationships: is_a meiosis II [GO:0007135]; is a type of male meiotic nuclear division [GO:0007140]